{
  "gene_name": "Putative UPF0633 protein MGC21881",
  "gene_symbol": "A6NN06",
  "term_id": "UNKNOWN:0002",
  "term_label": "Unknown biological process",
  "gene": "UniProtKB:A6NN06"
}